magnesium ion transmembrane transport [GO:1903830] (biological process) Subtypes: GO:0045016, GO:0160176 Definition: The directed movement of magnesium ion across a membrane. Relationships: is_a magnesium ion transport [GO:0015693]; is a type of monoatomic cation transmembrane transport [GO:0098655] References: PMID:11254124 Sources: GOC:TermGenie, GO_REF:0000069